{
  "gene_name": "V-set and transmembrane domain-containing protein 2-like protein",
  "term_label": "Unknown biological process",
  "gene_symbol": "VSTM2L",
  "term_id": "UNKNOWN:0002",
  "gene": "UniProtKB:Q96N03"
}